{
  "gene": "UniProtKB:P62851",
  "term_id": "UNKNOWN:0002",
  "term_label": "Unknown biological process",
  "gene_symbol": "RPS25",
  "gene_name": "Small ribosomal subunit protein eS25"
}